{
  "term_label": "cell-cell signaling",
  "gene_name": "Gap junction alpha-10 protein",
  "gene": "UniProtKB:Q969M2",
  "term_id": "GO:0007267",
  "gene_symbol": "GJA10"
}